{
  "term_label": "extracellular space",
  "gene": "UniProtKB:P01148",
  "gene_name": "Progonadoliberin-1",
  "gene_symbol": "GNRH1",
  "term_id": "GO:0005615"
}